{
  "gene_name": "UPF0690 protein C1orf52",
  "term_label": "Unknown biological process",
  "term_id": "UNKNOWN:0002",
  "gene": "UniProtKB:Q8N6N3",
  "gene_symbol": "C1orf52"
}